{
  "gene_name": "Zinc finger protein interacting with ribonucleoprotein K",
  "term_id": "GO:0000978",
  "gene_symbol": "ZIK1",
  "term_label": "RNA polymerase II cis-regulatory region sequence-specific DNA binding",
  "gene": "UniProtKB:Q3SY52"
}